{
  "gene": "UniProtKB:Q96AJ9",
  "term_id": "GO:0031201",
  "gene_symbol": "VTI1A",
  "term_label": "SNARE complex",
  "gene_name": "Vesicle transport through interaction with t-SNAREs homolog 1A"
}